{
  "term_id": "UNKNOWN:0002",
  "gene_name": "Cocaine esterase",
  "gene_symbol": "CES2",
  "term_label": "Unknown biological process",
  "gene": "UniProtKB:O00748"
}